{
  "gene_name": "Zinc finger protein 627",
  "gene_symbol": "ZNF627",
  "term_label": "RNA polymerase II transcription regulatory region sequence-specific DNA binding",
  "term_id": "GO:0000977",
  "gene": "UniProtKB:Q7L945"
}